negative regulation of cell proliferation involved in contact inhibition [GO:0060244] (biological process) Definition: Any process that stops, prevents or reduces the rate or extent of cell proliferation in response to cell density. Sources: GOC:dph Relationships: is a type of negative regulation of cell population proliferation [GO:0008285]; is part of contact inhibition [GO:0060242]